ribonucleoside bisphosphate biosynthetic process [GO:0034030] (biological process) Definition: The chemical reactions and pathways resulting in the formation of a ribonucleoside bisphosphate, a compound consisting of a nucleobase linked to a ribose sugar esterified with one phosphate group attached to each of two different hydroxyl groups on the sugar. Subtypes: GO:0034036 Relationships: is a type of nucleoside bisphosphate biosynthetic process [GO:0033866]; is a type of ribonucleoside bisphosphate metabolic process [GO:0033875] Sources: GOC:mah, GOC:pde Also known as: ribonucleoside bisphosphate anabolism, ribonucleoside bisphosphate biosynthesis, ribonucleoside bisphosphate formation, ribonucleoside bisphosphate synthesis